{
  "term_id": "GO:0030154",
  "term_label": "cell differentiation",
  "gene": "UniProtKB:O00571",
  "gene_name": "ATP-dependent RNA helicase DDX3X",
  "gene_symbol": "DDX3X"
}